{
  "term_id": "GO:0006974",
  "term_label": "DNA damage response",
  "gene_symbol": "ETAA1",
  "gene": "UniProtKB:Q9NY74",
  "gene_name": "Ewing's tumor-associated antigen 1"
}